swimming behavior [GO:0036269] (BP) Relationships: is a type of locomotory behavior [GO:0007626] Also known as: swimming behaviour Definition: The response to external or internal stimuli that results in the locomotory process of swimming. Swimming is the self-propelled movement of an organism through the water. References: PMID:16764679 Sources: GOC:cvs